{
  "gene_symbol": "SRPK3",
  "gene": "UniProtKB:Q9UPE1",
  "term_label": "intracellular signal transduction",
  "term_id": "GO:0035556",
  "gene_name": "SRSF protein kinase 3"
}